{
  "gene": "UniProtKB:P41217",
  "gene_symbol": "CD200",
  "gene_name": "OX-2 membrane glycoprotein",
  "term_label": "axon",
  "term_id": "GO:0030424"
}